intercellular bridge [GO:0045171] (cellular component) Definition: A direct connection between the cytoplasm of two cells that is formed following the completion of cleavage furrow ingression during cell division. They are usually present only briefly prior to completion of cytokinesis. However, in some cases, such as the bridges between germ cells during their development, they become stabilised. References: PMID:9635420 Relationships: is a type of cellular anatomical structure [GO:0110165] Subtypes: germline ring canal [GO:0045172], somatic ring canal [GO:0098549]